{
  "gene": "UniProtKB:O95947",
  "term_label": "chromatin",
  "term_id": "GO:0000785",
  "gene_symbol": "TBX6",
  "gene_name": "T-box transcription factor TBX6"
}